negative regulation of eosinophil differentiation [GO:0045644] (biological process) Also known as: down regulation of eosinophil differentiation, down-regulation of eosinophil differentiation, downregulation of eosinophil differentiation, inhibition of eosinophil differentiation Relationships: is a type of negative regulation of granulocyte differentiation [GO:0030853]; is a type of regulation of eosinophil differentiation [GO:0045643]; negatively regulates GO:0030222 Sources: GOC:go_curators Definition: Any process that stops, prevents, or reduces the frequency, rate or extent of eosinophil differentiation.